{
  "gene_name": "High affinity cAMP-specific and IBMX-insensitive 3',5'-cyclic phosphodiesterase 8B",
  "term_label": "negative regulation of cAMP/PKA signal transduction",
  "term_id": "GO:0141162",
  "gene": "UniProtKB:O95263",
  "gene_symbol": "PDE8B"
}